glycine reductase complex [GO:0030700] (cellular component) Relationships: is a type of oxidoreductase complex [GO:1990204]; is part of GO:0005737 Definition: Complex that possesses glycine reductase activity; usually comprises three subunits, of which two are selenoproteins; the subunits are typically designated selenoprotein A, selenoprotein B and protein C. References: PMID:2018775 Sources: GOC:mah Note: Note that this term represents a location and not a function; the activity possessed by this complex is mentioned in the definition for the purpose of describing and distinguishing the complex. The function possessed by this complex is represented by the molecular function term 'glycine reductase activity ; GO:0030699'.